{
  "term_label": "serine-type endopeptidase activity",
  "term_id": "GO:0004252",
  "gene_name": "Vitamin K-dependent protein C",
  "gene_symbol": "PROC",
  "gene": "UniProtKB:P04070"
}